{
  "gene": "UniProtKB:Q5VZ66",
  "gene_symbol": "JAKMIP3",
  "term_id": "UNKNOWN:0002",
  "term_label": "Unknown biological process",
  "gene_name": "Janus kinase and microtubule-interacting protein 3"
}